{
  "gene": "UniProtKB:Q9BW61",
  "gene_symbol": "DDA1",
  "term_label": "Unknown molecular function",
  "term_id": "UNKNOWN:0001",
  "gene_name": "DET1- and DDB1-associated protein 1"
}